vegetative phase change [GO:0010050] (biological process) Definition: Any process involved in the transition of a plant from a juvenile phase of vegetative development to an adult phase of vegetative development. Sources: GOC:tb Relationships: is a type of post-embryonic development [GO:0009791] Regulation: RO_0002211 by GO:0010321